macropinocytic cup membrane [GO:0070686] (cellular component) Sources: GOC:mah Definition: The portion of the plasma membrane surrounding a macropinocytic cup. Also known as: crown membrane Relationships: is a type of GO:0031253; is part of macropinocytic cup [GO:0070685]